{
  "gene_name": "Anaphase-promoting complex subunit 11",
  "gene": "UniProtKB:Q9NYG5",
  "term_label": "nucleus",
  "gene_symbol": "ANAPC11",
  "term_id": "GO:0005634"
}